regulation of excitatory synapse assembly [GO:1904889] (BP) Definition: Any process that modulates the frequency, rate or extent of excitatory synapse assembly. Sources: GOC:PARL, GOC:TermGenie, GOC:bf, GO_REF:0000058 Subtypes: regulation of postsynaptic density assembly [GO:0099151], GO:1904890, positive regulation of excitatory synapse assembly [GO:1904891] Also known as: regulation of excitatory synapse formation Relationships: is a type of regulation of synapse assembly [GO:0051963]; regulates excitatory synapse assembly [GO:1904861]